{
  "gene_symbol": "MGAT5B",
  "term_label": "Golgi apparatus",
  "gene": "UniProtKB:Q3V5L5",
  "term_id": "GO:0005794",
  "gene_name": "Alpha-1,6-mannosylglycoprotein 6-beta-N-acetylglucosaminyltransferase B"
}